{
  "gene": "UniProtKB:Q8WWY6",
  "gene_name": "Methyl-CpG-binding domain protein 3-like 1",
  "term_id": "GO:0000122",
  "term_label": "negative regulation of transcription by RNA polymerase II",
  "gene_symbol": "MBD3L1"
}